{
  "gene_symbol": "SLBP",
  "gene_name": "Histone RNA hairpin-binding protein",
  "term_id": "GO:0006398",
  "term_label": "mRNA 3'-end processing by stem-loop binding and cleavage",
  "gene": "UniProtKB:Q14493"
}